negative regulation of smooth muscle cell-matrix adhesion [GO:2000098] (biological process) Definition: Any process that stops, prevents, or reduces the frequency, rate or extent of smooth muscle cell-matrix adhesion. Sources: GOC:BHF Relationships: is_a negative regulation of cell-matrix adhesion [GO:0001953]; is a type of regulation of smooth muscle cell-matrix adhesion [GO:2000097]; negatively regulates smooth muscle cell-matrix adhesion [GO:0061302]